{
  "gene_name": "Protein cereblon",
  "term_id": "UNKNOWN:0001",
  "gene": "UniProtKB:Q96SW2",
  "gene_symbol": "CRBN",
  "term_label": "Unknown molecular function"
}